L-lactate dehydrogenase activity [GO:0140171] (molecular function) Sources: GOC:pg Definition: Catalysis of the reaction: (S)-lactate + A = AH(2) + pyruvate. Relationships: is a type of lactate dehydrogenase activity [GO:0004457] Subtypes: L-lactate dehydrogenase (NAD+) activity [GO:0004459], L-lactate dehydrogenase (cytochrome) activity [GO:0004460]